follicle-stimulating hormone receptor binding [GO:0031762] (molecular function) Definition: Binding to a follicle-stimulating hormone receptor. Relationships: is a type of G protein-coupled receptor binding [GO:0001664] Also known as: FSH receptor binding, follicle stimulating hormone receptor binding, follicle stimulating hormone receptor ligand Sources: GOC:mah, GOC:nln